{
  "gene_symbol": "OR56B2",
  "gene": "UniProtKB:Q8NGI1",
  "term_id": "GO:0005886",
  "term_label": "plasma membrane",
  "gene_name": "Putative olfactory receptor 56B2"
}